{
  "gene": "UniProtKB:O60512",
  "term_label": "galactosyltransferase activity",
  "gene_name": "Beta-1,4-galactosyltransferase 3",
  "gene_symbol": "B4GALT3",
  "term_id": "GO:0008378"
}